{
  "gene_name": "Keratin, type I cuticular Ha6",
  "term_label": "structural constituent of skin epidermis",
  "term_id": "GO:0030280",
  "gene_symbol": "KRT36",
  "gene": "UniProtKB:O76013"
}